positive regulation of zoospore formation [GO:0075241] (biological process) Definition: Any process that activates, maintains or increases the frequency, rate or extent of zoospore formation, a process in which a diploid cell undergoes meiosis, and the meiotic products acquire specialized features of asexual motile mononucleate flagellated spores called zoospores. Sources: GOC:pamgo_curators Relationships: is a type of GO:0075240; is a type of positive regulation of sporangiospore formation [GO:0075287]; positively regulates GO:0075239